{
  "gene_name": "Regulator of chromosome condensation",
  "term_label": "guanyl-nucleotide exchange factor activity",
  "gene": "UniProtKB:P18754",
  "term_id": "GO:0005085",
  "gene_symbol": "RCC1"
}